{
  "term_label": "meiotic nuclear membrane microtubule tethering complex",
  "gene_symbol": "KASH5",
  "gene_name": "Protein KASH5",
  "term_id": "GO:0034993",
  "gene": "UniProtKB:Q8N6L0"
}